L-asparagine catabolic process via 2-oxosuccinamate [GO:0033346] (biological process) Sources: GOC:mah, MetaCyc:PWY-4002 Definition: The chemical reactions and pathways resulting in the breakdown of L-asparagine, via the intermediate 2-oxosuccinamate. Relationships: is a type of L-asparagine catabolic process [GO:0006530]